{
  "gene_name": "Ubiquitin carboxyl-terminal hydrolase 15",
  "gene": "UniProtKB:Q9Y4E8",
  "term_label": "Unknown molecular function",
  "gene_symbol": "USP15",
  "term_id": "UNKNOWN:0001"
}